{
  "term_id": "UNKNOWN:0002",
  "gene_symbol": "S100G",
  "term_label": "Unknown biological process",
  "gene": "UniProtKB:P29377",
  "gene_name": "Protein S100-G"
}